{
  "gene_symbol": "STOML1",
  "term_label": "plasma membrane",
  "gene_name": "Stomatin-like protein 1",
  "gene": "UniProtKB:Q9UBI4",
  "term_id": "GO:0005886"
}